{
  "gene_name": "Centrosomal protein of 19 kDa",
  "gene": "UniProtKB:Q96LK0",
  "term_id": "GO:0005814",
  "term_label": "centriole",
  "gene_symbol": "CEP19"
}